{
  "gene_symbol": "NPAS2",
  "gene_name": "Neuronal PAS domain-containing protein 2",
  "term_label": "DNA-binding transcription factor activity, RNA polymerase II-specific",
  "gene": "UniProtKB:Q99743",
  "term_id": "GO:0000981"
}